prenol kinase activity [GO:0052673] (molecular function) Sources: GOC:ai, GOC:kd Definition: Catalysis of the reaction: prenol + nucleoside triphosphate = prenyl phosphate + nucleoside diphosphate activity. Also known as: prenol phosphotransferase activity, prenyl alcohol kinase activity, prenyl alcohol phosphotransferase activity Relationships: is a type of phosphotransferase activity, alcohol group as acceptor [GO:0016773]